{
  "term_label": "positive regulation of phosphatidylinositol 3-kinase/protein kinase B signal transduction",
  "gene_name": "Tyrosine-protein kinase receptor UFO",
  "gene_symbol": "AXL",
  "term_id": "GO:0051897",
  "gene": "UniProtKB:P30530"
}